{
  "gene_name": "Probable phospholipid-transporting ATPase IIB",
  "term_label": "plasma membrane",
  "gene_symbol": "ATP9B",
  "term_id": "GO:0005886",
  "gene": "UniProtKB:O43861"
}